{
  "gene_symbol": "RUSC1-AS1",
  "term_label": "Unknown cellular component",
  "term_id": "UNKNOWN:0003",
  "gene_name": "Putative uncharacterized protein RUSC1-AS1",
  "gene": "UniProtKB:Q66K80"
}